nematode pharynx development [GO:0160094] (biological process) References: PMID:18050503 Relationships: is_a GO:0060465 Definition: The process whose specific outcome is the progression of nematode pharynx over time, from its formation to the mature structure.